response to host redox environment [GO:0075137] (biological process) Relationships: is a type of GO:0075136 Also known as: response of symbiont to host redox environment Note: Note that this term is used to annotate gene products of the symbiont. Definition: Any process that results in a change in state or activity of the symbiont organism or its cell (in terms of movement, secretion, enzyme production, gene expression, etc.) as a result of detecting the redox environment in host organism. The host is defined as the larger of the organisms involved in a symbiotic interaction. Sources: GOC:pamgo_curators